{
  "gene": "UniProtKB:Q86VI1",
  "term_id": "GO:0000149",
  "gene_name": "Exocyst complex component 3-like protein",
  "term_label": "SNARE binding",
  "gene_symbol": "EXOC3L1"
}